{
  "gene": "UniProtKB:Q9Y5X9",
  "term_label": "high-density lipoprotein particle remodeling",
  "gene_symbol": "LIPG",
  "term_id": "GO:0034375",
  "gene_name": "Endothelial lipase"
}